{
  "term_id": "UNKNOWN:0001",
  "gene_symbol": "SLC10A7",
  "gene_name": "Sodium_bile acid cotransporter 7",
  "gene": "UniProtKB:Q0GE19",
  "term_label": "Unknown molecular function"
}